{
  "gene_symbol": "ERBIN",
  "gene_name": "Erbin",
  "term_id": "GO:0035556",
  "term_label": "intracellular signal transduction",
  "gene": "UniProtKB:Q96RT1"
}